{
  "term_label": "protein O-linked glycosylation",
  "gene_symbol": "GALNT3",
  "gene_name": "Polypeptide N-acetylgalactosaminyltransferase 3",
  "term_id": "GO:0006493",
  "gene": "UniProtKB:Q14435"
}